{
  "term_id": "GO:0005856",
  "gene_symbol": "CCDC110",
  "gene": "UniProtKB:Q8TBZ0",
  "gene_name": "Coiled-coil domain-containing protein 110",
  "term_label": "cytoskeleton"
}